{
  "gene_symbol": "LAMB2",
  "term_label": "extracellular space",
  "term_id": "GO:0005615",
  "gene_name": "Laminin subunit beta-2",
  "gene": "UniProtKB:P55268"
}